{
  "gene": "UniProtKB:Q8WU49",
  "gene_symbol": "C7orf33",
  "gene_name": "Uncharacterized protein C7orf33",
  "term_id": "UNKNOWN:0001",
  "term_label": "Unknown molecular function"
}